{
  "gene_name": "DNA damage-induced apoptosis suppressor protein",
  "term_label": "nucleus",
  "gene": "UniProtKB:Q8IXT1",
  "gene_symbol": "DDIAS",
  "term_id": "GO:0005634"
}